negative regulation of telomere maintenance in response to DNA damage [GO:1904506] (biological process) Definition: Any process that stops, prevents or reduces the frequency, rate or extent of telomere maintenance in response to DNA damage. References: PMID:22579284 Sources: GOC:BHF, GOC:BHF_telomere, GOC:TermGenie, GOC:nc, GO_REF:0000058 Also known as: down regulation of DNA damage response, telomere maintenance, down regulation of telomere maintenance in response to DNA damage, down-regulation of DNA damage response, telomere maintenance, down-regulation of telomere maintenance in response to DNA damage, downregulation of DNA damage response, telomere maintenance, downregulation of telomere maintenance in response to DNA damage, negative regulation of DNA damage response, telomere maintenance, inhibition of DNA damage response, telomere maintenance, inhibition of telomere maintenance in response to DNA damage Relationships: is a type of GO:0032205; is a type of GO:0048585; is a type of GO:1904505; negatively regulates telomere maintenance in response to DNA damage [GO:0043247] Subtypes: GO:1905765